{
  "gene": "UniProtKB:A8MU46",
  "term_label": "Unknown cellular component",
  "gene_name": "Smoothelin-like protein 1",
  "term_id": "UNKNOWN:0003",
  "gene_symbol": "SMTNL1"
}